{
  "term_label": "Unknown biological process",
  "term_id": "UNKNOWN:0002",
  "gene_symbol": "SLC9B1",
  "gene": "UniProtKB:Q4ZJI4",
  "gene_name": "Sodium_hydrogen exchanger 9B1"
}